pilus [GO:0009289] (cellular component) Relationships: is a type of GO:0042995 Definition: A proteinaceous hair-like appendage on the surface of bacteria ranging from 2-8 nm in diameter. Also known as: fimbria, fimbriae, fimbrium, pili References: PMID:28496159 Sources: GOC:pamgo_curators Subtypes: type IV pilus [GO:0044096], curli [GO:0098774], type I pilus [GO:0140621]